lipoprotein localization to membrane [GO:0044873] (biological process) Sources: GOC:jl Subtypes: lipoprotein localization to outer membrane [GO:0044874] Definition: A process in which a lipoprotein is transported to, or maintained in, a specific location in a membrane. Relationships: is a type of lipoprotein localization [GO:0044872]; is a type of GO:0051668